{
  "gene_symbol": "GBP2",
  "gene_name": "Guanylate-binding protein 2",
  "term_label": "GTP binding",
  "term_id": "GO:0005525",
  "gene": "UniProtKB:P32456"
}